{
  "term_id": "GO:0019722",
  "gene": "UniProtKB:O00574",
  "gene_symbol": "CXCR6",
  "term_label": "calcium-mediated signaling",
  "gene_name": "C-X-C chemokine receptor type 6"
}